{
  "term_id": "GO:0072546",
  "term_label": "EMC complex",
  "gene_symbol": "EMC10",
  "gene_name": "ER membrane protein complex subunit 10",
  "gene": "UniProtKB:Q5UCC4"
}